{
  "term_label": "Unknown biological process",
  "gene": "UniProtKB:A0A590UJ96",
  "gene_name": "Uncharacterized protein",
  "term_id": "UNKNOWN:0002",
  "gene_symbol": "LOC122526780"
}